{
  "gene_symbol": "WASF2",
  "gene_name": "Actin-binding protein WASF2",
  "gene": "UniProtKB:Q9Y6W5",
  "term_label": "positive regulation of Arp2/3 complex-mediated actin nucleation",
  "term_id": "GO:2000601"
}